{
  "gene_name": "Dehydrogenase_reductase SDR family member on chromosome X",
  "gene_symbol": "DHRSX",
  "gene": "UniProtKB:Q8N5I4",
  "term_label": "Unknown molecular function",
  "term_id": "UNKNOWN:0001"
}